{
  "gene": "UniProtKB:A0A0K0K1C4",
  "term_id": "GO:0007166",
  "gene_name": "T cell receptor beta variable 27",
  "term_label": "cell surface receptor signaling pathway",
  "gene_symbol": "TRBV27"
}